{
  "gene_name": "cGMP-dependent 3',5'-cyclic phosphodiesterase",
  "gene": "UniProtKB:O00408",
  "term_id": "GO:0010754",
  "term_label": "negative regulation of receptor guanylyl cyclase signaling pathway",
  "gene_symbol": "PDE2A"
}